fusion of sperm to egg plasma membrane involved in double fertilization forming two zygotes [GO:0061935] (biological process) Relationships: is a type of cellular process involved in reproduction in multicellular organism [GO:0022412]; is_a plasma membrane fusion [GO:0045026]; is part of double fertilization forming two zygotes [GO:0009677] Definition: The binding and fusion of a sperm, with the plasma membrane of the oocyte as part of the process of double fertilization forming two zygotes. Sources: GOC:dph